{
  "term_id": "UNKNOWN:0001",
  "gene": "UniProtKB:P02810",
  "term_label": "Unknown molecular function",
  "gene_symbol": "PRH2",
  "gene_name": "Salivary acidic proline-rich phosphoprotein 1_2"
}